TRAPPII protein complex [GO:1990071] (cellular component) Definition: A complex that mediates intra-Golgi traffic, Golgi exit, endosome-to-Golgi traffic, and the trafficking of autophagy proteins from Golgi to the phagophore assembly site. Binds to a component of the COPI coat. In yeast it includes the following subunits: Bet3 (as homodimer), Bet5, Tca17, Trs20, Trs23, Trs31, Trs33, Trs65, Trs120, Trs130. The whole complex is thought to dimerize with itself. References: PMID:20375281, PMID:22669257 Sources: GOC:bhm Relationships: is a type of TRAPP complex [GO:0030008]; is part of endosome [GO:0005768]; is part of Golgi apparatus [GO:0005794]